chloride channel regulator activity [GO:0017081] (molecular function) Relationships: is a type of GO:0099106; regulates GO:0005254 Definition: Binds to and modulates the activity of a chloride channel. Subtypes: chloride channel inhibitor activity [GO:0019869] Sources: GOC:mah